L-valine-2-oxoglutarate transaminase activity [GO:0052655] (molecular function) Definition: Catalysis of the reaction: 2-oxoglutarate + L-valine = 3-methyl-2-oxobutanoic acid + L-glutamatic acid. Sources: RHEA:24813 Also known as: L-valine aminotransferase activity Relationships: is a type of branched-chain-amino-acid transaminase activity [GO:0004084]